Wnt receptor recycling [GO:0038019] (biological process) References: PMID:19643732 Sources: GOC:bf, GOC:signaling Definition: The process that results in the return of a Wnt receptor to an active state at the plasma membrane. An active state is when the receptor is ready to receive a Wnt signal. Internalized Wnt receptors can be recycled to the plasma membrane or sorted to lysosomes for protein degradation. Also known as: Frizzled recycling Relationships: is a type of GO:0001881; is part of positive regulation of Wnt signaling pathway [GO:0030177]